{
  "gene": "UniProtKB:P06850",
  "gene_name": "Corticoliberin",
  "term_id": "GO:0070093",
  "term_label": "negative regulation of glucagon secretion",
  "gene_symbol": "CRH"
}